mitotic metaphase chromosome alignment [GO:0007080] (biological process) Definition: A chromosome localization process whereby chromosomes are positioned in a specific order and orientation at the metaphase plate (spindle equator), during mitotic chromosome segregation. This alignment ensures that each daughter cell will receive the correct number of chromosomes during cell division. Relationships: is_a metaphase chromosome alignment [GO:0051310]; is_a GO:1903047; is part of mitotic sister chromatid segregation [GO:0000070] Sources: ISBN:0815316194